{
  "gene_symbol": "KIF18A",
  "gene_name": "Kinesin-like protein KIF18A",
  "term_label": "mitotic spindle astral microtubule",
  "term_id": "GO:0061673",
  "gene": "UniProtKB:Q8NI77"
}